right anterior basal body [GO:1902672] (cellular component) Definition: Any ciliary basal body that is part of a right anterior flagellum found in Giardia species (trophozoite stage). References: PMID:16607022, PMID:5961344 Sources: GOC:TermGenie, GOC:giardia, GO_REF:0000064, ISBN:9780124260207 Also known as: cilial basal body of right anterior cilium, cilial basal body of right anterior flagellum, ciliary basal body of right anterior cilium, ciliary basal body of right anterior flagellum, cilium basal body of right anterior cilium, cilium basal body of right anterior flagellum, microtubule basal body of right anterior cilium, microtubule basal body of right anterior flagellum, right anterior flagellum ciliary basal body Note: Note that we deem cilium and microtubule-based flagellum to be equivalent. Also note that, due to the asymmetric nature of the Giardia trophozoite, this term is defined spatially as the trophozoite is viewed from the dorsal side, with the two nuclei dorsal to the ventral disc, and the ventral disc toward the anterior. Relationships: is a type of ciliary basal body [GO:0036064]; is part of right anterior flagellum [GO:0097555]